{
  "gene_name": "Golgin subfamily A member 8J",
  "gene_symbol": "GOLGA8J",
  "gene": "UniProtKB:A6NMD2",
  "term_label": "Golgi cis cisterna",
  "term_id": "GO:0000137"
}